{
  "gene_name": "Tubby-related protein 2",
  "term_label": "Unknown molecular function",
  "gene": "UniProtKB:O00295",
  "term_id": "UNKNOWN:0001",
  "gene_symbol": "TULP2"
}